meiotic spindle disassembly [GO:0051229] (biological process) Relationships: is a type of meiotic spindle organization [GO:0000212]; is a type of GO:0051230 Also known as: meiotic spindle breakdown, meiotic spindle catabolism, meiotic spindle degradation, spindle breakdown during meiosis, spindle degradation during meiosis, spindle disassembly during meiosis Definition: The controlled breakdown of the spindle during a meiotic cell cycle. Sources: GOC:ai